{
  "term_label": "Unknown biological process",
  "gene": "UniProtKB:I3L1E1",
  "gene_name": "Uncharacterized protein C19orf84",
  "gene_symbol": "C19orf84",
  "term_id": "UNKNOWN:0002"
}